response to interleukin-7 [GO:0098760] (biological process) Relationships: is a type of response to cytokine [GO:0034097] Sources: GOC:BHF, GOC:mah Subtypes: cellular response to interleukin-7 [GO:0098761] Definition: Any process that results in a change in state or activity of a cell or an organism (in terms of movement, secretion, enzyme production, gene expression, etc.) as a result of an interleukin-7 stimulus. Also known as: response to IL-7